{
  "term_label": "phosphatidylinositol-4,5-bisphosphate phospholipase C activity",
  "term_id": "GO:0004435",
  "gene": "UniProtKB:Q9UPR0",
  "gene_symbol": "PLCL2",
  "gene_name": "Inactive phospholipase C-like protein 2"
}